{
  "term_id": "GO:0010460",
  "gene_name": "Pro-adrenomedullin",
  "term_label": "positive regulation of heart rate",
  "gene_symbol": "ADM",
  "gene": "UniProtKB:P35318"
}